{
  "gene_name": "AP-3 complex subunit mu-2",
  "gene_symbol": "AP3M2",
  "gene": "UniProtKB:P53677",
  "term_label": "Golgi to vacuole transport",
  "term_id": "GO:0006896"
}